{
  "term_id": "GO:0005161",
  "term_label": "platelet-derived growth factor receptor binding",
  "gene": "UniProtKB:P01127",
  "gene_symbol": "PDGFB",
  "gene_name": "Platelet-derived growth factor subunit B"
}